C-methyltransferase activity [GO:0008169] (molecular function) Sources: GOC:ai Definition: Catalysis of the transfer of a methyl group to the carbon atom of an acceptor molecule. Subtypes: tRNA (adenine(37)-C2)-methyltransferase activity [GO:0002935], sterol 24-C-methyltransferase activity [GO:0003838], uroporphyrin-III C-methyltransferase activity [GO:0004851], 2-methoxy-6-polyprenyl-1,4-benzoquinol methyltransferase activity [GO:0008425], GO:0009383, GO:0035244, deoxycytidylate C-methyltransferase activity [GO:0050003], 2-phytyl-1,4-naphthoquinone methyltransferase activity [GO:0052624], rRNA (adenine(2503)-C2-)-methyltransferase activity [GO:0070040], rRNA (uridine-C5-)-methyltransferase activity [GO:0070041] Relationships: is a type of methyltransferase activity [GO:0008168]